signal peptide processing [GO:0006465] (biological process) Definition: The proteolytic removal of a signal peptide from a protein during or after transport to a specific location in the cell. Also known as: leader peptide processing Subtypes: SRP-dependent cotranslational protein targeting to membrane, signal sequence processing [GO:0006618] References: PMID:31214988 Sources: GOC:mah Relationships: is a type of protein processing [GO:0016485]